positive regulation of calcium-independent cell-cell adhesion [GO:0051041] (biological process) Also known as: up regulation of calcium-independent cell-cell adhesion, up-regulation of calcium-independent cell-cell adhesion, upregulation of calcium-independent cell-cell adhesion, activation of calcium-independent cell-cell adhesion, stimulation of calcium-independent cell-cell adhesion Sources: GOC:ai Relationships: is a type of positive regulation of cell-cell adhesion [GO:0022409]; is a type of regulation of calcium-independent cell-cell adhesion [GO:0051040]; positively regulates calcium-independent cell-cell adhesion [GO:0016338] Definition: Any process that activates or increases the frequency, rate or extent of calcium-independent cell-cell adhesion.